{
  "term_label": "CXCR chemokine receptor binding",
  "gene": "UniProtKB:P42830",
  "term_id": "GO:0045236",
  "gene_name": "C-X-C motif chemokine 5",
  "gene_symbol": "CXCL5"
}